{
  "term_label": "adenylate cyclase-activating G protein-coupled receptor signaling pathway",
  "term_id": "GO:0007189",
  "gene": "UniProtKB:P01258",
  "gene_symbol": "CALCA",
  "gene_name": "Calcitonin"
}